{
  "gene_symbol": "NPHS1",
  "term_id": "GO:0098609",
  "gene": "UniProtKB:O60500",
  "term_label": "cell-cell adhesion",
  "gene_name": "Nephrin"
}